melanosome localization [GO:0032400] (biological process) Relationships: is a type of pigment granule localization [GO:0051875] Sources: GOC:ln Subtypes: melanosome transport [GO:0032402] Definition: Any process in which a melanosome is transported to, and/or maintained in, a specific location within the cell. Also known as: melanosome localisation